{
  "gene_name": "Serine_threonine-protein kinase 26",
  "term_label": "protein serine/threonine kinase activity",
  "term_id": "GO:0004674",
  "gene_symbol": "STK26",
  "gene": "UniProtKB:Q9P289"
}